tooth mineralization [GO:0034505] (biological process) Definition: The process in which calcium salts are deposited into calcareous tooth structures such as dental enamel, dentin and cementum. Sources: GOC:mah, MP:0002817, MSH:D014074 Also known as: tooth calcification Relationships: is a type of biomineral tissue development [GO:0031214]; BFO_0000050 GO:0042476 Regulation: regulated by regulation of tooth mineralization [GO:0070170]; negatively regulated by negative regulation of tooth mineralization [GO:0070171]; positively regulated by GO:0070172 Subtypes: enamel mineralization [GO:0070166], GO:0071529, GO:0097188